trophectodermal cell differentiation [GO:0001829] (biological process) Definition: The process in which a relatively unspecialized cell acquires the specialized features of a trophectoderm cell. Also known as: trophectoderm cell differentiation Note: See also the Anatomical Dictionary for Mouse Development ontology terms 'TS4, trophectoderm ; EMAP:19'. Relationships: is a type of cell differentiation [GO:0030154]; is part of GO:0001825 Sources: GOC:dph, ISBN:0124020607, ISBN:0198542771